2,5-didehydrogluconate reductase activity [GO:0050580] (MF) Also known as: 2,5-diketo-D-gluconate reductase activity, 2-dehydro-D-gluconate:NADP+ 2-oxidoreductase activity, YqhE reductase Relationships: is a type of oxidoreductase activity, acting on the CH-OH group of donors, NAD or NADP as acceptor [GO:0016616] Sources: EC:1.1.1.274, MetaCyc:1.1.1.274-RXN Definition: Catalysis of the reaction: 2-dehydro-D-gluconate + NADP+ = 2,5-didehydro-D-gluconate + NADPH + H+.